budding cell apical bud growth [GO:0007118] (biological process) Sources: GOC:go_curators Definition: Growth at the tip of a bud, in a cell that reproduces by budding. Regulation: regulated by regulation of budding cell apical bud growth [GO:0010568] Also known as: apical bud growth Relationships: is a type of GO:0007117